protein acylation [GO:0043543] (biological process) Sources: GOC:jl Also known as: protein amino acid acylation Subtypes: protein acetylation [GO:0006473], GO:0018190, protein formylation [GO:0018256], GO:0018335, protein palmitoylation [GO:0018345], protein myristoylation [GO:0018377], protein malonylation [GO:0044394], GO:0045234, protein decanoylation [GO:0051366], GO:0061921, peptidyl-lysine glutarylation [GO:0106227], peptidyl-lysine crotonylation [GO:0140066], peptidyl-lysine butyrylation [GO:0140067] Relationships: is_a protein modification process [GO:0036211] Definition: The addition of an acyl group, any group or radical of the form RCO- where R is an organic group, to a protein amino acid.